{
  "gene_symbol": "SIRPG",
  "gene_name": "Signal-regulatory protein gamma",
  "term_id": "UNKNOWN:0001",
  "gene": "UniProtKB:Q9P1W8",
  "term_label": "Unknown molecular function"
}